hepatic stellate cell differentiation [GO:0061521] (biological process) References: PMID:9407545 Sources: GOC:dph Definition: The process in which a relatively unspecialized cell acquires the specialized structural and/or functional features of a hepatic stellate cell. Relationships: is a type of cell differentiation [GO:0030154]